negative regulation of ecdysone receptor signaling pathway [GO:0120143] (biological process) Also known as: negative regulation of ecdysone receptor-mediated signaling pathway References: PMID:23072462 Sources: GOC:ha Relationships: is a type of negative regulation of intracellular steroid hormone receptor signaling pathway [GO:0033144]; is_a regulation of ecdysone receptor signaling pathway [GO:0120141]; is a type of negative regulation of cellular response to alcohol [GO:1905958]; negatively regulates ecdysone receptor signaling pathway [GO:0035076] Definition: Any process that stops, prevents, or reduces the frequency, rate or extent of any ecdysone receptor signaling pathway.